{
  "term_id": "GO:0005634",
  "term_label": "nucleus",
  "gene_name": "Transcription factor Sp7",
  "gene_symbol": "SP7",
  "gene": "UniProtKB:Q8TDD2"
}